regulation of endothelial microparticle formation [GO:2000335] (biological process) Also known as: regulation of endothelial microparticle generation, regulation of endothelial microparticle release Subtypes: GO:2000336, positive regulation of endothelial microparticle formation [GO:2000337] Relationships: is a type of regulation of blood microparticle formation [GO:2000332]; regulates endothelial microparticle formation [GO:0072565] Sources: GOC:BHF, GOC:mah Definition: Any process that modulates the frequency, rate or extent of endothelial microparticle formation.